{
  "gene_symbol": "TECR",
  "gene": "UniProtKB:Q9NZ01",
  "term_id": "GO:0005783",
  "gene_name": "Very-long-chain enoyl-CoA reductase",
  "term_label": "endoplasmic reticulum"
}